regulation of protein tyrosine kinase activity [GO:0061097] (biological process) Sources: GOC:dph, GOC:tb Subtypes: positive regulation of protein tyrosine kinase activity [GO:0061098], negative regulation of protein tyrosine kinase activity [GO:0061099] Relationships: is a type of regulation of protein kinase activity [GO:0045859]; is a type of GO:0050730; regulates protein tyrosine kinase activity [GO:0004713] Definition: Any process that modulates the rate, frequency, or extent of protein tyrosine kinase activity.